{
  "term_label": "Unknown biological process",
  "gene": "UniProtKB:Q9Y237",
  "gene_name": "Peptidyl-prolyl cis-trans isomerase NIMA-interacting 4",
  "gene_symbol": "PIN4",
  "term_id": "UNKNOWN:0002"
}